{
  "term_label": "anatomical structure morphogenesis",
  "gene_name": "Forkhead box protein D4-like 5",
  "gene": "UniProtKB:Q5VV16",
  "term_id": "GO:0009653",
  "gene_symbol": "FOXD4L5"
}